{
  "term_label": "signal recognition particle binding",
  "gene": "UniProtKB:P08240",
  "gene_name": "Signal recognition particle receptor subunit alpha",
  "term_id": "GO:0005047",
  "gene_symbol": "SRPRA"
}